S-methylmethionine-homocysteine S-methyltransferase activity [GO:0061627] (molecular function) Also known as: S-methylmethionine homocysteine transmethylase activity, homocysteine methyltransferase activity, homocysteine transmethylase activity, methylmethionine:homocysteine methyltransferase activity Relationships: is a type of S-methyltransferase activity [GO:0008172] Sources: RHEA:26337 Definition: Catalysis of the reaction: S-methyl-L-methionine + L-homocysteine = 2 L-methionine + H+.